establishment of bipolar cell polarity [GO:0061171] (biological process) Subtypes: cell growth mode switching, monopolar to bipolar [GO:0051523], establishment of bipolar cell polarity involved in cell morphogenesis [GO:0061159] Relationships: is a type of establishment of cell polarity [GO:0030010] Definition: The specification and formation of bipolar intracellular organization or cell growth patterns. Bipolar organization is the organization that is a mirror image along an axis from a plane. Sources: GOC:dph, GOC:vw Regulation: regulated by regulation of establishment of bipolar cell polarity [GO:0061172]; positively regulated by positive regulation of establishment of bipolar cell polarity [GO:0061173]; negatively regulated by negative regulation of establishment of bipolar cell polarity [GO:1904846]